{
  "term_label": "protein-glutamine gamma-glutamyltransferase activity",
  "gene_symbol": "EPB42",
  "gene_name": "Protein 4.2",
  "term_id": "GO:0003810",
  "gene": "UniProtKB:P16452"
}